{
  "gene": "UniProtKB:O60613",
  "term_label": "endoplasmic reticulum lumen",
  "gene_name": "Selenoprotein F",
  "gene_symbol": "SELENOF",
  "term_id": "GO:0005788"
}